{
  "gene_symbol": "CEP68",
  "gene": "UniProtKB:Q76N32",
  "term_label": "Unknown biological process",
  "gene_name": "Centrosomal protein of 68 kDa",
  "term_id": "UNKNOWN:0002"
}